{
  "gene_symbol": "JMJD4",
  "gene": "UniProtKB:Q9H9V9",
  "term_label": "nucleus",
  "term_id": "GO:0005634",
  "gene_name": "2-oxoglutarate and iron-dependent oxygenase JMJD4"
}